mannose-1-phosphate guanylyltransferase (GDP) activity [GO:0008928] (molecular function) Also known as: GDP:mannose-1-phosphate guanylyltransferase activity, GDP mannose phosphorylase activity, GDP-mannose 1-phosphate guanylyltransferase activity, GDP-mannose phosphorylase activity, GDP-mannose pyrophosphorylase activity, GDP:D-mannose-1-phosphate guanylyltransferase activity, GDP:alpha-D-mannose-1-phosphate guanylyltransferase activity, guanosine diphosphate-mannose 1-phosphate guanylyltransferase activity, guanosine diphosphomannose phosphorylase activity, mannose 1-phosphate (guanosine diphosphate) guanylyltransferase activity, mannose 1-phosphate guanylyltransferase activity Definition: Catalysis of the reaction: alpha-D-mannose 1-phosphate + GDP + H+ = GDP-alpha-D-mannose + phosphate. Sources: RHEA:12905 Relationships: is a type of GO:0070568